regulation of organelle assembly [GO:1902115] (biological process) Subtypes: regulation of cytoplasmic mRNA processing body assembly [GO:0010603], regulation of centriole replication [GO:0046599], regulation of stress granule assembly [GO:0062028], regulation of pseudohyphal septin ring assembly [GO:0062164], regulation of podosome assembly [GO:0071801], regulation of spindle assembly [GO:0090169], regulation of kinetochore assembly [GO:0090234], regulation of postsynaptic specialization assembly [GO:0099150], GO:1900503, regulation of cilium assembly [GO:1902017], negative regulation of organelle assembly [GO:1902116], positive regulation of organelle assembly [GO:1902117], GO:1902208, regulation of extracellular exosome assembly [GO:1903551], regulation of gut granule assembly [GO:1904755], GO:1905304, regulation of autophagosome assembly [GO:2000785] Relationships: is a type of regulation of organelle organization [GO:0033043]; is_a regulation of cellular component biogenesis [GO:0044087]; regulates organelle assembly [GO:0070925] Definition: Any process that modulates the frequency, rate or extent of organelle assembly. Sources: GOC:TermGenie, GOC:pr